{
  "term_id": "GO:0005737",
  "gene": "UniProtKB:Q9UNP9",
  "gene_name": "Peptidyl-prolyl cis-trans isomerase E",
  "term_label": "cytoplasm",
  "gene_symbol": "PPIE"
}